{
  "term_id": "UNKNOWN:0002",
  "gene": "UniProtKB:P62753",
  "gene_symbol": "RPS6",
  "term_label": "Unknown biological process",
  "gene_name": "Small ribosomal subunit protein eS6"
}